{
  "term_id": "UNKNOWN:0003",
  "term_label": "Unknown cellular component",
  "gene_symbol": "WDFY3",
  "gene": "UniProtKB:Q8IZQ1",
  "gene_name": "WD repeat and FYVE domain-containing protein 3"
}